peroxisomal importomer complex [GO:1990429] (cellular component) Relationships: is a type of GO:1990351 Definition: A protein complex responsible for transporting proteins into the peroxisomal matrix. An example of this complex is Pex14 found in S. cerevisae which has 9 core components and 12 transient interaction partners. Also known as: peroxisomal import pore, peroxisomal protein import machinery, Pex14 complex, Pex17p-Pex14p docking complex References: PMID:12667447, PMID:20154681, PMID:22375831